positive regulation of pre-miRNA processing [GO:2000633] (biological process) Sources: GOC:dph, GOC:sl Also known as: positive regulation of miRNA maturation, positive regulation of pre-microRNA processing Relationships: is a type of positive regulation of miRNA processing [GO:1903800]; is a type of regulation of pre-miRNA processing [GO:2000631]; positively regulates GO:0031054 Definition: Any process that activates or increases the frequency, rate or extent of pre-microRNA processing.